{
  "gene": "UniProtKB:P31358",
  "term_id": "UNKNOWN:0001",
  "gene_symbol": "CD52",
  "gene_name": "CAMPATH-1 antigen",
  "term_label": "Unknown molecular function"
}